{
  "gene_name": "Osteomodulin",
  "gene_symbol": "OMD",
  "gene": "UniProtKB:Q99983",
  "term_id": "UNKNOWN:0001",
  "term_label": "Unknown molecular function"
}